{
  "gene_symbol": "CWF19L1",
  "gene": "UniProtKB:Q69YN2",
  "gene_name": "CWF19-like protein 1",
  "term_label": "RNA lariat debranching enzyme activator activity",
  "term_id": "GO:0061632"
}